{
  "gene": "UniProtKB:Q9UNH5",
  "term_id": "GO:0072686",
  "gene_name": "Dual specificity protein phosphatase CDC14A",
  "term_label": "mitotic spindle",
  "gene_symbol": "CDC14A"
}